protein localization to basal ectoplasmic specialization [GO:0120145] (biological process) Definition: A process in which a protein is transported to, or maintained in, a location within a basal ectoplasmic specialization. Relationships: is_a protein localization to cell-cell junction [GO:0150105] Also known as: protein localisation in basal ectoplasmic specialization, protein localisation to basal ectoplasmic specialization, protein localization in basal ectoplasmic specialization References: PMID:22872576